arylamine glucosyltransferase activity [GO:0047684] (molecular function) Relationships: is a type of UDP-glucosyltransferase activity [GO:0035251] Also known as: UDP glucose-arylamine glucosyltransferase activity, UDP-glucose:arylamine N-D-glucosyltransferase activity, UDPglucose:arylamine N-D-glucosyltransferase activity, uridine diphosphoglucose-arylamine glucosyltransferase activity Definition: Catalysis of the reaction: UDP-glucose + an arylamine = UDP + an N-D-glucosylarylamine. Sources: EC:2.4.1.71, MetaCyc:ARYLAMINE-GLUCOSYLTRANSFERASE-RXN